glucan 1,4-alpha-maltotriohydrolase activity [GO:0033934] (molecular function) Sources: EC:3.2.1.116 Also known as: 1,4-alpha-D-glucan maltotriohydrolase activity, exo-maltotriohydrolase activity, maltotriohydrolase activity Definition: Catalysis of the hydrolysis of (1->4)-alpha-D-glucosidic linkages in amylaceous polysaccharides, to remove successive maltotriose residues from the non-reducing chain ends. Relationships: is a type of hydrolase activity, hydrolyzing O-glycosyl compounds [GO:0004553]